chemokine (C-C motif) ligand 21 binding [GO:0035758] (molecular function) Also known as: CCL21 binding Relationships: is a type of GO:0019957 Definition: Binding to chemokine (C-C motif) ligand 21. Sources: GOC:BHF